{
  "gene_name": "Glypican-1",
  "gene": "UniProtKB:P35052",
  "term_label": "regulation of protein localization to membrane",
  "term_id": "GO:1905475",
  "gene_symbol": "GPC1"
}